{
  "term_label": "plasma membrane",
  "gene_name": "Glycoprotein Xg",
  "term_id": "GO:0005886",
  "gene": "UniProtKB:P55808",
  "gene_symbol": "XG"
}